C-22 sterol desaturase (NADPH) activity [GO:0000249] (MF) Sources: EC:1.14.19.41 Relationships: is a type of sterol desaturase activity [GO:0070704] Definition: Catalysis of the reaction: 5-dehydroepisterol + H+ + NADPH + O2 = ergosta-5,7,22,24(28)-tetraen-3beta-ol + 2 H2O + NADP+. This reaction is the introduction of a double bond between the C-22 and C-23 carbons of certain sterols. Also converts sitosterol and 24-epi-campesterol to stigmasterol and brassicasterol, respectively.